negative regulation of natural killer cell proliferation [GO:0032818] (biological process) Relationships: is a type of negative regulation of natural killer cell activation [GO:0032815]; is a type of GO:0032817; is a type of negative regulation of lymphocyte proliferation [GO:0050672]; negatively regulates natural killer cell proliferation [GO:0001787] Sources: GOC:mah Also known as: down regulation of natural killer cell proliferation, down-regulation of natural killer cell proliferation, downregulation of natural killer cell proliferation, negative regulation of NK cell proliferation, inhibition of natural killer cell proliferation Definition: Any process that stops, prevents, or reduces the frequency, rate or extent of natural killer cell proliferation. Subtypes: GO:0032821